{
  "gene_name": "Endogenous retrovirus group K member 11 Pol protein",
  "gene_symbol": "ERVK-11",
  "gene": "UniProtKB:Q9UQG0",
  "term_label": "RNA stem-loop binding",
  "term_id": "GO:0035613"
}